{
  "gene_name": "Protein ARV1",
  "term_label": "sterol metabolic process",
  "term_id": "GO:0016125",
  "gene_symbol": "ARV1",
  "gene": "UniProtKB:Q9H2C2"
}